{
  "term_label": "mitochondrion",
  "gene": "UniProtKB:Q9BPW8",
  "gene_symbol": "NIPSNAP1",
  "gene_name": "Protein NipSnap homolog 1",
  "term_id": "GO:0005739"
}